{
  "term_label": "Unknown biological process",
  "gene_name": "Neutral cholesterol ester hydrolase 1",
  "term_id": "UNKNOWN:0002",
  "gene_symbol": "NCEH1",
  "gene": "UniProtKB:Q6PIU2"
}